plastid translation [GO:0032544] (biological process) Sources: GOC:go_curators Relationships: is a type of translation [GO:0006412]; is a type of GO:0009657; occurs in plastid [GO:0009536] Also known as: plastid protein anabolism, plastid protein biosynthesis, plastid protein formation, plastid protein synthesis, plastid protein translation Definition: The chemical reactions and pathways resulting in the formation of a protein in a plastid. This is a ribosome-mediated process in which the information in messenger RNA (mRNA) is used to specify the sequence of amino acids in the protein; the plastid has its own ribosomes and transfer RNAs, and uses a genetic code that differs from the nuclear code.